{
  "term_label": "mitochondrial respiratory chain complex I assembly",
  "gene": "UniProtKB:Q96CU9",
  "gene_name": "FAD-dependent oxidoreductase domain-containing protein 1",
  "gene_symbol": "FOXRED1",
  "term_id": "GO:0032981"
}